antipodal cell differentiation [GO:0009557] (biological process) Regulation: regulated by regulation of antipodal cell differentiation [GO:0045688]; negatively regulated by negative regulation of antipodal cell differentiation [GO:0045689]; positively regulated by GO:0045690 Relationships: is a type of cell differentiation [GO:0030154]; is part of megagametogenesis [GO:0009561] Definition: The process in which an uncellularized nucleus cellularizes and acquires the specialized features of an antipodal cell. Sources: GOC:jid, GOC:mtg_plant